{
  "gene_name": "Zinc finger protein 195",
  "term_id": "UNKNOWN:0003",
  "gene": "UniProtKB:O14628",
  "gene_symbol": "ZNF195",
  "term_label": "Unknown cellular component"
}